subset_property [oboInOwl#SubsetProperty]